{
  "gene_name": "Trinucleotide repeat-containing gene 6A protein",
  "term_id": "GO:0060213",
  "gene_symbol": "TNRC6A",
  "gene": "UniProtKB:Q8NDV7",
  "term_label": "positive regulation of nuclear-transcribed mRNA poly(A) tail shortening"
}